proline-rich region binding [GO:0070064] (molecular function) Relationships: is_a protein binding [GO:0005515] Sources: GOC:mah Definition: Binding to a proline-rich region, i.e. a region that contains a high proportion of proline residues, in a protein.